V(D)J recombination [GO:0033151] (biological process) Definition: The process in which immune receptor V, D, and J, or V and J gene segments, depending on the specific receptor, are recombined within a single locus utilizing the conserved heptamer and nonomer recombination signal sequences (RSS). Relationships: is a type of somatic diversification of immune receptors via germline recombination within a single locus [GO:0002562] Sources: GOC:add, ISBN:0781700221, ISBN:0781735149 Also known as: V(D)J joining, V-D-J joining, V-D-J recombination, V-J joining, V-J recombination Subtypes: GO:0033152, GO:0033153